host-mediated suppression of viral proces [GO:0044793] (biological process) Subtypes: host-mediated suppression of viral transcription [GO:0043922], negative regulation by host of viral glycoprotein metabolic process [GO:0044871] Relationships: is a type of host-mediated perturbation of viral process [GO:0044788] Sources: GOC:jl Definition: A process in which a host organism interferes with, inhibits or disrupts a process being mediated by a virus with which it is infected. Also known as: negative regulation by host of viral process